{
  "gene_symbol": "ACTA1",
  "gene": "UniProtKB:P68133",
  "term_label": "actin filament",
  "gene_name": "Actin, alpha skeletal muscle",
  "term_id": "GO:0005884"
}